{
  "term_id": "GO:0030317",
  "gene_name": "Spermatid maturation protein 1",
  "gene_symbol": "SPEM1",
  "term_label": "flagellated sperm motility",
  "gene": "UniProtKB:Q8N4L4"
}